{
  "gene": "UniProtKB:Q96FZ2",
  "term_id": "GO:0097681",
  "gene_symbol": "HMCES",
  "term_label": "double-strand break repair via alternative nonhomologous end joining",
  "gene_name": "Abasic site processing protein HMCES"
}